{
  "term_label": "cytoplasm",
  "gene": "UniProtKB:Q9NRH3",
  "gene_name": "Tubulin gamma-2 chain",
  "gene_symbol": "TUBG2",
  "term_id": "GO:0005737"
}